regulation of fever generation by prostaglandin secretion [GO:0100009] (biological process) Relationships: is a type of prostaglandin secretion [GO:0032310]; regulates fever generation [GO:0001660] Sources: GOC:cjm, GOC:obol Regulation: regulated by regulation of fever generation by regulation of prostaglandin secretion [GO:0071810] Subtypes: GO:0100011 Definition: Any prostaglandin secretion process that regulates fever generation.